positive regulation of amine metabolic process [GO:0033240] (biological process) Definition: Any process that activates or increases the frequency, rate or extent of the chemical reactions and pathways involving amines. Also known as: positive regulation of amine metabolism, positive regulation of cellular amine metabolic process Relationships: is_a GO:0009893; is_a regulation of amine metabolic process [GO:0033238]; positively regulates GO:0009308 Subtypes: GO:0033243, positive regulation of dopamine metabolic process [GO:0045964], GO:0060409, positive regulation of methane biosynthetic process from dimethylamine [GO:1900320], positive regulation of methane biosynthetic process from trimethylamine [GO:1900332], positive regulation of methane biosynthetic process from methylamine [GO:1900350], positive regulation of spermidine biosynthetic process [GO:1901307] Sources: GOC:mah